{
  "gene_name": "Cellular tumor antigen p53",
  "term_label": "RNA polymerase II cis-regulatory region sequence-specific DNA binding",
  "term_id": "GO:0000978",
  "gene": "UniProtKB:P04637",
  "gene_symbol": "TP53"
}